CTDK-1 complex [GO:0070692] (CC) Relationships: is a type of GO:0008024 References: PMID:16721054, PMID:19328067 Sources: GOC:mah, GOC:vw Definition: A positive transcription elongation factor complex that comprises the CDK kinase CTK1 (in budding yeast), Lsk1 (in fission yeast) (corresponding to the Panther PTHR24056:SF39 family), a cyclin and an additional gamma subunit (corresponding to the InterPRO entry IPR024638). Also known as: C-terminal domain kinase I complex, CTDK-I complex, Ctk complex, trimeric positive transcription elongation factor complex b